{
  "gene_symbol": "TFAP2A",
  "term_id": "GO:0042127",
  "gene": "UniProtKB:P05549",
  "gene_name": "Transcription factor AP-2-alpha",
  "term_label": "regulation of cell population proliferation"
}